export from cell [GO:0140352] (BP) Definition: The directed movement of some substance from a cell, into the extracellular region. This may occur via transport across the plasma membrane or via exocytosis. Subtypes: GO:0032940, xenobiotic export from cell [GO:0046618], export across plasma membrane [GO:0140115], lipid export from cell [GO:0140353], migracytosis [GO:0140495] Sources: GOC:pg Relationships: is a type of transport [GO:0006810]; is a type of cellular process [GO:0009987] Also known as: efflux